fruit ripening, non-climacteric [GO:0009837] (biological process) Relationships: is a type of fruit ripening [GO:0009835] Definition: A fruit ripening process that does not involve a respiratory burst. Sources: GOC:lr, ISBN:0521587840